SHREC complex localization [GO:0072688] (biological process) Definition: Any process in which a SHREC complex is transported to, or maintained in, a specific location. Sources: GOC:mah Also known as: SHREC complex localisation, establishment and maintenance of SHREC complex localization Relationships: is a type of protein-containing complex localization [GO:0031503]